{
  "gene_name": "C-C chemokine receptor type 1",
  "gene_symbol": "CCR1",
  "gene": "UniProtKB:P32246",
  "term_label": "C-C chemokine receptor activity",
  "term_id": "GO:0016493"
}